{
  "gene_name": "Tumor necrosis factor ligand superfamily member 12",
  "gene_symbol": "TNFSF12",
  "term_label": "cytokine activity",
  "gene": "UniProtKB:O43508",
  "term_id": "GO:0005125"
}